{
  "gene_symbol": "KRT14",
  "term_label": "keratin filament",
  "term_id": "GO:0045095",
  "gene": "UniProtKB:P02533",
  "gene_name": "Keratin, type I cytoskeletal 14"
}